negative regulation of thioredoxin peroxidase activity by peptidyl-threonine phosphorylation [GO:1903125] (biological process) Definition: A peptidyl-threonine phosphorylation that results in negative regulation of thioredoxin peroxidase activity. References: PMID:21850687 Sources: GOC:PARL, GOC:TermGenie, GOC:bf, GO_REF:0000063 Also known as: negative regulation of TPx activity by peptidyl-threonine phosphorylation, negative regulation of TrxPx activity by peptidyl-threonine phosphorylation, negative regulation of thiol peroxidase activity by peptidyl-threonine phosphorylation Relationships: is a type of GO:0018107; negatively regulates thioredoxin peroxidase activity [GO:0008379]